positive regulation of neural retina development [GO:0061075] (biological process) Relationships: is a type of GO:0061074; is a type of positive regulation of retina development in camera-type eye [GO:1902868]; positively regulates GO:0003407 Definition: Any process that increases the rate, frequency, or extent of neural retina development, the progression of the neural retina over time from its initial formation to the mature structure. The neural retina is the part of the retina that contains neurons and photoreceptor cells. Sources: GOC:dph